myosin V binding [GO:0031489] (molecular function) References: PMID:11212351, PMID:33541831 Sources: GOC:mah Definition: Binding to a class V myosin; myosin V is a dimeric molecule involved in intracellular transport. Relationships: is a type of myosin binding [GO:0017022]